regulation of non-motile cilium assembly [GO:1902855] (BP) References: PMID:23807208 Sources: GOC:TermGenie, GOC:cilia, GOC:kmv, GO_REF:0000058 Also known as: regulation of immotile primary cilium assembly, regulation of nonmotile primary cilia assembly, regulation of nonmotile primary cilium assembly, regulation of sensory cilium assembly, regulation of sensory cilium biogenesis Definition: Any process that modulates the frequency, rate or extent of non-motile cilium assembly. Relationships: is a type of regulation of cilium assembly [GO:1902017]; regulates non-motile cilium assembly [GO:1905515] Subtypes: GO:1902856, GO:1902857